negative regulation of homotypic cell-cell adhesion [GO:0034111] (BP) Sources: GOC:add Relationships: is a type of negative regulation of cell-cell adhesion [GO:0022408]; is_a regulation of homotypic cell-cell adhesion [GO:0034110]; negatively regulates GO:0034109 Subtypes: negative regulation of erythrocyte aggregation [GO:0034119], GO:0090331 Definition: Any process that stops, prevents, or reduces the frequency, rate, or extent of homotypic cell-cell adhesion.